{
  "term_label": "Unknown molecular function",
  "term_id": "UNKNOWN:0001",
  "gene_symbol": "SCAMP5",
  "gene_name": "Secretory carrier-associated membrane protein 5",
  "gene": "UniProtKB:Q8TAC9"
}